{
  "gene_symbol": "SPOCK2",
  "term_id": "GO:0031012",
  "gene": "UniProtKB:Q92563",
  "gene_name": "Testican-2",
  "term_label": "extracellular matrix"
}